vitamin B6 biosynthetic process [GO:0042819] (biological process) Relationships: is a type of water-soluble vitamin biosynthetic process [GO:0042364]; is a type of vitamin B6 metabolic process [GO:0042816]; is a type of pyridine-containing compound biosynthetic process [GO:0072525] Subtypes: pyridoxine biosynthetic process [GO:0008615], pyridoxal biosynthetic process [GO:0042821], GO:0042823 Also known as: vitamin B6 anabolism, vitamin B6 biosynthesis, vitamin B6 formation, vitamin B6 synthesis, pyridoxine-5'-phosphate biosynthesis References: PMID:16157873, PMID:30671974 Sources: GOC:jl Definition: The chemical reactions and pathways resulting in the formation of any of the vitamin B6 compounds; pyridoxal, pyridoxamine and pyridoxine and the active form, pyridoxal phosphate.